deoxyribodipyrimidine photo-lyase activity [GO:0003904] (MF) Definition: Catalysis of the reaction: cyclobutadipyrimidine (in DNA) = 2 pyrimidine residues (in DNA). This reaction represents the reactivation of irradiated DNA by light. Relationships: is a type of GO:0003913 Also known as: CPD photolyase activity, deoxyribodipyrimidine photolyase activity, DNA cyclobutane dipyrimidine photolyase activity, DNA-photoreactivating enzyme, PRE, PhrB photolyase activity, deoxyribocyclobutadipyrimidine pyrimidine-lyase activity, deoxyribonucleate pyrimidine dimer lyase (photosensitive), deoxyribonucleic cyclobutane dipyrimidine photolyase activity, deoxyribonucleic photolyase activity, dipyrimidine photolyase (photosensitive), photolyase activity, photoreactivating enzyme activity, phr A photolyase activity Sources: EC:4.1.99.3